{
  "gene_name": "Kinesin heavy chain isoform 5C",
  "term_label": "ATP hydrolysis activity",
  "gene": "UniProtKB:O60282",
  "term_id": "GO:0016887",
  "gene_symbol": "KIF5C"
}